{
  "term_label": "cytosol",
  "gene_name": "AMP deaminase 2",
  "term_id": "GO:0005829",
  "gene": "UniProtKB:Q01433",
  "gene_symbol": "AMPD2"
}